{
  "term_id": "GO:0042063",
  "gene_symbol": "GCM2",
  "term_label": "gliogenesis",
  "gene": "UniProtKB:O75603",
  "gene_name": "Chorion-specific transcription factor GCMb"
}